regulation of protein localization to Cajal body [GO:1904869] (biological process) Also known as: regulation of protein localisation in Cajal body, regulation of protein localisation to Cajal body, regulation of protein localization in Cajal body References: PMID:25467444 Sources: GOC:BHF, GOC:BHF_telomere, GOC:TermGenie, GOC:nc, GO_REF:0000058 Relationships: is a type of regulation of protein localization to nucleus [GO:1900180]; regulates protein localization to Cajal body [GO:1904867] Definition: Any process that modulates the frequency, rate or extent of protein localization to Cajal body. Subtypes: negative regulation of protein localization to Cajal body [GO:1904870], GO:1904871